beta-endorphin binding [GO:0031626] (molecular function) Definition: Binding to beta-endorphin, a peptide generated by the cleavage of pro-opiomelanocortin. Relationships: is_a GO:0033218 References: PMID:6267560 Sources: GOC:nln